{
  "gene_symbol": "FOXO6",
  "gene": "UniProtKB:A8MYZ6",
  "term_label": "regulation of transcription by RNA polymerase II",
  "gene_name": "Forkhead box protein O6",
  "term_id": "GO:0006357"
}